{
  "term_label": "short-chain fatty acid catabolic process",
  "gene": "UniProtKB:P23141",
  "term_id": "GO:0019626",
  "gene_name": "Liver carboxylesterase 1",
  "gene_symbol": "CES1"
}